alanine racemase activity [GO:0008784] (molecular function) Also known as: L-alanine racemase activity Definition: Catalysis of the reaction: L-alanine = D-alanine. Sources: EC:5.1.1.1, RHEA:20249 Relationships: is_a amino-acid racemase activity [GO:0047661]